{
  "gene_name": "Dead end protein homolog 1",
  "term_id": "GO:0003729",
  "gene": "UniProtKB:Q8IYX4",
  "gene_symbol": "DND1",
  "term_label": "mRNA binding"
}